{
  "gene_name": "Sclerostin domain-containing protein 1",
  "term_id": "GO:0005615",
  "gene": "UniProtKB:Q6X4U4",
  "gene_symbol": "SOSTDC1",
  "term_label": "extracellular space"
}